response to topologically incorrect protein [GO:0035966] (biological process) Sources: GOC:bf Definition: Any process that results in a change in state or activity of a cell or an organism (in terms of movement, secretion, enzyme production, gene expression, etc.) as a result of a protein that is not folded in its correct three-dimensional structure. Relationships: is_a response to stress [GO:0006950] Subtypes: response to unfolded protein [GO:0006986], cellular response to topologically incorrect protein [GO:0035967], response to misfolded protein [GO:0051788] Also known as: response to misfolded or unfolded protein